{
  "term_id": "GO:0007605",
  "term_label": "sensory perception of sound",
  "gene_name": "Ankyrin repeat domain-containing protein 24",
  "gene_symbol": "ANKRD24",
  "gene": "UniProtKB:Q8TF21"
}